{
  "term_id": "GO:0005096",
  "gene_symbol": "TBC1D8",
  "term_label": "GTPase activator activity",
  "gene_name": "TBC1 domain family member 8",
  "gene": "UniProtKB:O95759"
}